{
  "gene_symbol": "ST6GAL1",
  "gene_name": "Beta-galactoside alpha-2,6-sialyltransferase 1",
  "gene": "UniProtKB:P15907",
  "term_label": "beta-galactoside alpha-2,6-sialyltransferase activity",
  "term_id": "GO:0003835"
}